{
  "gene": "UniProtKB:Q6QHC5",
  "gene_symbol": "DEGS2",
  "term_id": "GO:0042284",
  "gene_name": "Sphingolipid delta(4)-desaturase_C4-monooxygenase DES2",
  "term_label": "sphingolipid delta-4 desaturase activity"
}